{
  "gene_symbol": "OTUB2",
  "term_label": "Unknown biological process",
  "gene_name": "Ubiquitin thioesterase OTUB2",
  "gene": "UniProtKB:Q96DC9",
  "term_id": "UNKNOWN:0002"
}